{
  "gene": "UniProtKB:Q15653",
  "term_label": "cellular response to lipopolysaccharide",
  "gene_symbol": "NFKBIB",
  "term_id": "GO:0071222",
  "gene_name": "NF-kappa-B inhibitor beta"
}